guanylate cyclase inhibitor activity [GO:0030251] (molecular function) Sources: GOC:mah Relationships: is a type of cyclase inhibitor activity [GO:0010852]; is a type of guanylate cyclase regulator activity [GO:0030249]; negatively regulates guanylate cyclase activity [GO:0004383] Definition: Binds to and stops, prevents or reduces the activity of guanylate cyclase.